{
  "gene": "UniProtKB:Q96EF0",
  "term_label": "phosphatidylinositol-3-phosphate phosphatase activity",
  "gene_name": "Myotubularin-related protein 8",
  "term_id": "GO:0004438",
  "gene_symbol": "MTMR8"
}